{
  "term_id": "GO:0003725",
  "gene": "UniProtKB:Q7Z2E3",
  "gene_name": "Aprataxin",
  "term_label": "double-stranded RNA binding",
  "gene_symbol": "APTX"
}